{
  "gene_name": "Semaphorin-4B",
  "gene": "UniProtKB:Q9NPR2",
  "term_label": "positive regulation of cell migration",
  "term_id": "GO:0030335",
  "gene_symbol": "SEMA4B"
}